{
  "term_id": "GO:0000049",
  "gene_name": "L-seryl-tRNA(Sec) kinase",
  "term_label": "tRNA binding",
  "gene": "UniProtKB:Q8IV42",
  "gene_symbol": "PSTK"
}